{
  "gene": "UniProtKB:Q96A61",
  "term_id": "GO:0061630",
  "gene_symbol": "TRIM52",
  "gene_name": "E3 ubiquitin-protein ligase TRIM52",
  "term_label": "ubiquitin protein ligase activity"
}